regulation of cell communication involved in growth plate cartilage morphogenesis [GO:0003437] (biological process) Definition: Any process that modulates the frequency, rate or extent of cell communication that contributes to the shaping of the growth plate cartilage. Sources: GOC:ascb_2009, GOC:dph, GOC:tb Relationships: is a type of regulation of cell communication [GO:0010646]; is part of growth plate cartilage morphogenesis [GO:0003422]